host cell PML body [GO:0075341] (cellular component) Relationships: is a type of GO:0044094 Also known as: host cell PML NB, host cell PML nuclear body Sources: GOC:BHF, GOC:jl Definition: A nuclear body that reacts against SP100 auto-antibodies (PML = promyelocytic leukemia) located within a cell of a host organism.